cellular response to estrogen stimulus [GO:0071391] (biological process) Also known as: cellular response to oestrogen stimulus, cellular response to 17alpha-ethynylestradiol Sources: GOC:mah Relationships: is a type of cellular response to hormone stimulus [GO:0032870]; is a type of GO:0043627 Definition: Any process that results in a change in state or activity of a cell (in terms of movement, secretion, enzyme production, gene expression, etc.) as a result of stimulus by an estrogen, C18 steroid hormones that can stimulate the development of female sexual characteristics.